{
  "gene": "UniProtKB:Q96HA7",
  "term_id": "UNKNOWN:0001",
  "gene_symbol": "TONSL",
  "gene_name": "Tonsoku-like protein",
  "term_label": "Unknown molecular function"
}